{
  "term_id": "GO:0003678",
  "gene": "UniProtKB:Q9Y265",
  "gene_name": "RuvB-like 1",
  "term_label": "DNA helicase activity",
  "gene_symbol": "RUVBL1"
}